{
  "gene_symbol": "SLC12A7",
  "gene_name": "Solute carrier family 12 member 7",
  "term_label": "potassium:chloride symporter activity",
  "gene": "UniProtKB:Q9Y666",
  "term_id": "GO:0015379"
}